{
  "gene_symbol": "BNIP1",
  "term_label": "SNARE complex",
  "gene_name": "Vesicle transport protein SEC20",
  "term_id": "GO:0031201",
  "gene": "UniProtKB:Q12981"
}